{
  "gene_name": "Mitochondrial import inner membrane translocase subunit Tim21",
  "gene": "UniProtKB:Q9BVV7",
  "term_id": "GO:0030150",
  "gene_symbol": "TIMM21",
  "term_label": "protein import into mitochondrial matrix"
}